{
  "term_id": "GO:0050853",
  "gene_symbol": "BTK",
  "gene_name": "Tyrosine-protein kinase BTK",
  "gene": "UniProtKB:Q06187",
  "term_label": "B cell receptor signaling pathway"
}